PML body [GO:0016605] (CC) Relationships: is a type of nuclear body [GO:0016604] Also known as: ND10, PML NB, PML nuclear body, nuclear dot Definition: A class of nuclear body; they react against SP100 auto-antibodies (PML, promyelocytic leukemia); cells typically contain 10-30 PML bodies per nucleus; alterations in the localization of PML bodies occurs after viral infection. References: PMID:10944585 Sources: GOC:ma